cytoplasmic actin-based contraction involved in cell motility [GO:0060327] (biological process) Definition: The actin filament-based movement by which cytoplasmic actin filaments slide past one another resulting in a contraction that propels the cell from one place to another. Sources: GOC:dph Relationships: is a type of actin-mediated cell contraction [GO:0070252]; BFO_0000050 cell motility [GO:0048870] Subtypes: substrate-dependent cell migration, cell contraction [GO:0006932], GO:0060328, cytoplasmic actin-based contraction involved in rearward cell motility [GO:0060329]